{
  "term_label": "transcription elongation by RNA polymerase I",
  "gene": "UniProtKB:Q9GZS1",
  "term_id": "GO:0006362",
  "gene_name": "DNA-directed RNA polymerase I subunit RPA49",
  "gene_symbol": "POLR1E"
}